{
  "term_id": "GO:0002767",
  "gene": "UniProtKB:P43628",
  "term_label": "immune response-inhibiting cell surface receptor signaling pathway",
  "gene_name": "Killer cell immunoglobulin-like receptor 2DL3",
  "gene_symbol": "KIR2DL3"
}